putrescine transmembrane transporter activity [GO:0015489] (molecular function) Definition: Enables the transfer of putrescine from one side of a membrane to the other. Putrescine is 1,4-diaminobutane, the polyamine formed by decarboxylation of ornithine and the metabolic precursor of spermidine and spermine. Sources: GOC:ai Relationships: is a type of GO:0015203; BFO_0000050 putrescine transport [GO:0015847] Subtypes: GO:0015496, ABC-type putrescine transporter activity [GO:0015594], GO:0043861